{
  "gene_symbol": "SH3TC1",
  "term_label": "Unknown cellular component",
  "gene": "UniProtKB:Q8TE82",
  "term_id": "UNKNOWN:0003",
  "gene_name": "SH3 domain and tetratricopeptide repeat-containing protein 1"
}